{
  "gene_name": "Phospholipid scramblase family member 5",
  "term_id": "GO:0017128",
  "term_label": "phospholipid scramblase activity",
  "gene": "UniProtKB:A0PG75",
  "gene_symbol": "PLSCR5"
}